{
  "term_label": "regulation of microtubule cytoskeleton organization",
  "gene_symbol": "BICD2",
  "gene": "UniProtKB:Q8TD16",
  "term_id": "GO:0070507",
  "gene_name": "Protein bicaudal D homolog 2"
}